positive regulation of catecholamine secretion [GO:0033605] (biological process) Definition: Any process that activates or increases the frequency, rate or extent of the regulated release of a catecholamine. Sources: GOC:mah Also known as: up regulation of catecholamine secretion, up-regulation of catecholamine secretion, upregulation of catecholamine secretion, activation of catecholamine secretion, stimulation of catecholamine secretion Relationships: is a type of regulation of catecholamine secretion [GO:0050433]; is a type of positive regulation of amine transport [GO:0051954]; is a type of positive regulation of secretion by cell [GO:1903532]; positively regulates catecholamine secretion [GO:0050432] Subtypes: GO:0010701, positive regulation of epinephrine secretion [GO:0032812], positive regulation of dopamine secretion [GO:0033603]